{
  "term_id": "UNKNOWN:0001",
  "term_label": "Unknown molecular function",
  "gene_symbol": "ZNF223",
  "gene": "UniProtKB:Q9UK11",
  "gene_name": "Zinc finger protein 223"
}